5' transitive RNA interference [GO:1990514] (biological process) Relationships: is a type of transitive RNA interference [GO:0036453] References: PMID:24369430 Sources: GOC:pf Definition: An RNA interference where the silencing signal spreads 5' along the target mRNA, outside of the initial target sequence. Typically involves the formation of secondary siRNAs formed when the initial mRNA target sequence functions as a template for 5' to 3' synthesis of new dsRNA.